{
  "gene_name": "Putative zinc finger protein 727",
  "term_id": "GO:0006355",
  "term_label": "regulation of DNA-templated transcription",
  "gene_symbol": "ZNF727",
  "gene": "UniProtKB:A8MUV8"
}